{
  "term_label": "Unknown cellular component",
  "term_id": "UNKNOWN:0003",
  "gene": "UniProtKB:P36575",
  "gene_name": "Arrestin-C",
  "gene_symbol": "ARR3"
}